D-galacturonate biosynthetic process [GO:0033482] (biological process) Sources: GOC:jsg, GOC:mah Definition: The chemical reactions and pathways resulting in the formation of D-galacturonate, the D-enantiomer of galacturonate, the anion of galacturonic acid. Relationships: is a type of galacturonate biosynthetic process [GO:0033481]; is a type of monosaccharide biosynthetic process [GO:0046364]; is a type of D-galacturonate metabolic process [GO:0046396] Also known as: D-galacturonate anabolism, D-galacturonate biosynthesis, D-galacturonate formation, D-galacturonate synthesis